deoxycytidine biosynthetic process [GO:0046093] (biological process) Definition: The chemical reactions and pathways resulting in the formation of deoxycytidine, 2-deoxyribosylcytosine, one of the four major nucleosides of DNA. Sources: GOC:go_curators Also known as: deoxycytidine anabolism, deoxycytidine biosynthesis, deoxycytidine formation, deoxycytidine synthesis Relationships: is a type of GO:0046092; is a type of pyrimidine deoxyribonucleoside biosynthetic process [GO:0046126] Subtypes: deoxycytidine salvage [GO:0006237]